anthocyanin-containing compound catabolic process [GO:0046284] (biological process) Relationships: is a type of glycoside catabolic process [GO:0016139]; is a type of pigment catabolic process [GO:0046149]; is a type of flavonoid catabolic process [GO:0046275]; is a type of GO:0046283 Definition: The chemical reactions and pathways resulting in the breakdown of anthocyanins, any member of a group of intensely colored soluble glycosides of anthocyanidins. Regulation: regulated by GO:1900000; negatively regulated by GO:1900001; positively regulated by positive regulation of anthocyanin catabolic process [GO:1900002] Sources: GOC:ai Also known as: anthocyanin breakdown, anthocyanin catabolic process, anthocyanin catabolism, anthocyanin degradation